heme transport [GO:0015886] (biological process) Definition: The directed movement of heme, any compound of iron complexed in a porphyrin (tetrapyrrole) ring, into, out of or within a cell, or between cells, by means of some agent such as a transporter or pore. Subtypes: GO:0035351, GO:0097037, GO:0140420 Also known as: haem transport Sources: GOC:ai Relationships: is a type of GO:0071705; is a type of GO:1901678